{
  "gene_symbol": "OPTN",
  "gene_name": "Optineurin",
  "term_id": "GO:0034067",
  "gene": "UniProtKB:Q96CV9",
  "term_label": "protein localization to Golgi apparatus"
}